negative regulation of neurotrophin production [GO:0032900] (biological process) Subtypes: negative regulation of nerve growth factor production [GO:0032904] Also known as: down regulation of neurotrophin production, down-regulation of neurotrophin production, downregulation of neurotrophin production, inhibition of neurotrophin production Definition: Any process that stops, prevents, or reduces the frequency, rate, or extent of production of a neurotrophin. Relationships: is a type of GO:0032899; is a type of GO:0051241; negatively regulates neurotrophin production [GO:0032898] Sources: GOC:mah